{
  "gene_name": "Calponin-1",
  "gene_symbol": "CNN1",
  "term_id": "GO:0015629",
  "term_label": "actin cytoskeleton",
  "gene": "UniProtKB:P51911"
}